{
  "gene_symbol": "MEOX1",
  "term_id": "GO:0005634",
  "gene": "UniProtKB:P50221",
  "gene_name": "Homeobox protein MOX-1",
  "term_label": "nucleus"
}